{
  "gene_symbol": "USP17L10",
  "term_id": "GO:0042981",
  "term_label": "regulation of apoptotic process",
  "gene_name": "Ubiquitin carboxyl-terminal hydrolase 17-like protein 10",
  "gene": "UniProtKB:C9JJH3"
}